{
  "gene_symbol": "SCCPDH",
  "term_label": "Unknown molecular function",
  "gene": "UniProtKB:Q8NBX0",
  "term_id": "UNKNOWN:0001",
  "gene_name": "Saccharopine dehydrogenase-like oxidoreductase"
}